{
  "gene_name": "Zinc finger and SCAN domain-containing protein 18",
  "gene_symbol": "ZSCAN18",
  "term_label": "regulation of transcription by RNA polymerase II",
  "gene": "UniProtKB:Q8TBC5",
  "term_id": "GO:0006357"
}